{
  "gene_name": "Fibroblast growth factor 11",
  "gene": "UniProtKB:Q92914",
  "term_label": "nucleus",
  "term_id": "GO:0005634",
  "gene_symbol": "FGF11"
}